{
  "term_id": "GO:0007626",
  "term_label": "locomotory behavior",
  "gene": "UniProtKB:P83859",
  "gene_symbol": "QRFP",
  "gene_name": "Orexigenic neuropeptide QRFP"
}